{
  "gene_name": "Homeobox protein TGIF2",
  "term_id": "GO:0005634",
  "term_label": "nucleus",
  "gene": "UniProtKB:Q9GZN2",
  "gene_symbol": "TGIF2"
}